raffinose catabolic process [GO:0034484] (biological process) Definition: The chemical reactions and pathways resulting in the breakdown of raffinose, the trisaccharide beta-D-fructofuranosyl alpha-D-galactopyranosyl-(1->6)-alpha-D-glucopyranoside. Subtypes: GO:0036259 Relationships: is a type of oligosaccharide catabolic process [GO:0009313]; is a type of raffinose metabolic process [GO:0033530] Sources: GOC:mah Also known as: raffinose breakdown, raffinose catabolism, raffinose degradation